2,3-dihydroxybenzoate 3,4-dioxygenase activity [GO:0045133] (molecular function) Sources: EC:1.13.11.14, RHEA:18477 Relationships: is a type of oxidoreductase activity, acting on single donors with incorporation of molecular oxygen, incorporation of two atoms of oxygen [GO:0016702] Definition: Catalysis of the reaction: 2,3-dihydroxybenzoate + O2 = 2-hydroxy-3-(3-oxoprop-1-enyl)but-2-enedioate + H+. Also known as: 2,3-dihydroxybenzoate 1,2-dioxygenase activity, 2,3-dihydroxybenzoate oxygenase activity, 2,3-dihydroxybenzoate:oxygen 3,4-oxidoreductase (decyclizing), 2,3-dihydroxybenzoic oxygenase activity, o-pyrocatechuate oxygenase activity